arsenate ion transmembrane transport [GO:1901684] (biological process) Note: Note that this term is not intended for use in annotating lateral movement within membranes. Sources: GOC:TermGenie Definition: The process in which arsenate is transported across a membrane. Relationships: is a type of arsenite transport [GO:0015700]; is a type of transmembrane transport [GO:0055085]